response to sodium dodecyl sulfate [GO:0072706] (biological process) Definition: Any process that results in a change in state or activity of a cell or an organism (in terms of movement, secretion, enzyme production, gene expression, etc.) as a result of a sodium dodecyl sulfate (SDS) stimulus. Sources: GOC:mah Also known as: response to SDS Relationships: is a type of GO:1901700 Subtypes: GO:0072707